{
  "gene_name": "Probable ATP-dependent RNA helicase DDX49",
  "gene_symbol": "DDX49",
  "gene": "UniProtKB:Q9Y6V7",
  "term_label": "nucleus",
  "term_id": "GO:0005634"
}